{
  "gene_name": "Solute carrier family 22 member 4",
  "term_label": "Unknown cellular component",
  "term_id": "UNKNOWN:0003",
  "gene": "UniProtKB:Q9H015",
  "gene_symbol": "SLC22A4"
}